diphenyl phthalate binding [GO:0035274] (molecular function) Definition: Binding to diphenyl phthalate, C(20)H(14)O(4). References: PMID:34697989 Also known as: DPP binding Relationships: is a type of binding [GO:0005488]